{
  "gene_name": "PHD finger protein 23",
  "term_label": "nucleus",
  "gene": "UniProtKB:Q9BUL5",
  "gene_symbol": "PHF23",
  "term_id": "GO:0005634"
}